{
  "term_id": "GO:1902108",
  "term_label": "regulation of mitochondrial membrane permeability involved in apoptotic process",
  "gene": "UniProtKB:Q5T1C6",
  "gene_symbol": "THEM4",
  "gene_name": "Acyl-coenzyme A thioesterase THEM4"
}